phthalate 4,5-cis-dihydrodiol dehydrogenase activity [GO:0018517] (molecular function) Sources: EC:1.3.1.64, RHEA:13837 Also known as: cis-4,5-dihydroxycyclohexa-1(6),2-diene-1,2-dicarboxylate:NAD+ oxidoreductase activity Relationships: is a type of oxidoreductase activity, acting on the CH-CH group of donors, NAD or NADP as acceptor [GO:0016628] Definition: Catalysis of the reaction: cis-4,5-dihydroxycyclohexa-2,6-diene-1,2-dicarboxylate + NAD+ = 4,5-dihydroxyphthalate + H+ + NADH.